{
  "gene_symbol": "GHRH",
  "gene_name": "Somatoliberin",
  "term_label": "peptide hormone receptor binding",
  "gene": "UniProtKB:P01286",
  "term_id": "GO:0051428"
}